meiotic anaphase II [GO:0007138] (BP) Definition: The cell cycle phase during which chromosomes separate and migrate towards the poles of the spindle the as part of meiosis II. Sources: GOC:mtg_cell_cycle Relationships: is a type of meiosis II cell cycle phase [GO:0098765]; is part of anaphase [GO:0051322]; is part of GO:0051327 Note: Note that this term should not be used for direct annotation. If you are trying to make an annotation to x phase, it is likely that the correct annotation is 'regulation of x/y phase transition' or to a process which occurs during the reported phase (i.e mitotic DNA replication for mitotic S-phase). To capture the phase when a specific location or process is observed, the phase term can be used in an annotation extension (PMID:24885854) applied to a cellular component term (with the relation exists_during) or a biological process term (with the relation happens_during).